{
  "term_id": "UNKNOWN:0002",
  "gene_name": "MAPK-interacting and spindle-stabilizing protein-like",
  "term_label": "Unknown biological process",
  "gene": "UniProtKB:Q8NDC0",
  "gene_symbol": "MAPK1IP1L"
}